{
  "gene_name": "Transient receptor potential cation channel subfamily M member 1",
  "term_id": "GO:0005886",
  "term_label": "plasma membrane",
  "gene": "UniProtKB:Q7Z4N2",
  "gene_symbol": "TRPM1"
}